{
  "term_label": "ceramide 1-phosphate transfer activity",
  "gene_name": "Ceramide transfer protein",
  "gene_symbol": "CERT1",
  "gene": "UniProtKB:Q9Y5P4",
  "term_id": "GO:1902388"
}